{
  "gene_name": "Golgi integral membrane protein 4",
  "gene_symbol": "GOLIM4",
  "gene": "UniProtKB:O00461",
  "term_id": "UNKNOWN:0001",
  "term_label": "Unknown molecular function"
}